flavonoid biosynthetic process [GO:0009813] (biological process) Definition: The chemical reactions and pathways resulting in the formation of flavonoids, a group of phenolic derivatives containing a flavan skeleton. Sources: GOC:tair_curators, ISBN:0198547684 Also known as: flavonoid anabolism, flavonoid biosynthesis, flavonoid formation, flavonoid synthesis Relationships: is a type of biosynthetic process [GO:0009058]; is a type of flavonoid metabolic process [GO:0009812] Subtypes: flavonoid phytoalexin biosynthetic process [GO:0009716], anthocyanin-containing compound biosynthetic process [GO:0009718], cyanidin 3-O-glucoside biosynthetic process [GO:0033485], delphinidin 3-O-glucoside biosynthetic process [GO:0033486], pelargonidin 3-O-glucoside biosynthetic process [GO:0033487], aurone biosynthetic process [GO:0051551], flavone biosynthetic process [GO:0051553] Regulation: regulated by regulation of flavonoid biosynthetic process [GO:0009962]; positively regulated by GO:0009963; negatively regulated by GO:0009964